{
  "gene": "UniProtKB:O60762",
  "term_label": "dolichyl-phosphate beta-D-mannosyltransferase activity",
  "gene_symbol": "DPM1",
  "gene_name": "Dolichol-phosphate mannosyltransferase subunit 1",
  "term_id": "GO:0004582"
}